{
  "gene_name": "Histamine H3 receptor",
  "term_id": "GO:0030594",
  "gene": "UniProtKB:Q9Y5N1",
  "term_label": "neurotransmitter receptor activity",
  "gene_symbol": "HRH3"
}